{
  "gene_name": "Actin-related protein 8",
  "gene_symbol": "ACTR8",
  "term_label": "Ino80 complex",
  "gene": "UniProtKB:Q9H981",
  "term_id": "GO:0031011"
}